{
  "term_id": "GO:0030301",
  "gene_symbol": "APOA2",
  "gene_name": "Apolipoprotein A-II",
  "term_label": "cholesterol transport",
  "gene": "UniProtKB:P02652"
}